{
  "gene": "UniProtKB:Q9UI17",
  "gene_name": "Dimethylglycine dehydrogenase, mitochondrial",
  "term_label": "mitochondrion",
  "gene_symbol": "DMGDH",
  "term_id": "GO:0005739"
}